{
  "gene": "UniProtKB:Q9BRP8",
  "gene_name": "Partner of Y14 and mago",
  "term_id": "GO:0035145",
  "gene_symbol": "PYM1",
  "term_label": "exon-exon junction complex"
}